{
  "gene": "UniProtKB:Q8IZD9",
  "term_label": "small GTPase binding",
  "term_id": "GO:0031267",
  "gene_symbol": "DOCK3",
  "gene_name": "Dedicator of cytokinesis protein 3"
}